lipid localization [GO:0010876] (biological process) Definition: Any process in which a lipid is transported to, or maintained in, a specific location. Sources: GOC:BHF, GOC:dph, GOC:tb Also known as: lipid localisation Relationships: is a type of GO:0033036 Regulation: RO_0002211 by regulation of lipid localization [GO:1905952]; negatively regulated by negative regulation of lipid localization [GO:1905953]; positively regulated by positive regulation of lipid localization [GO:1905954] Subtypes: lipid droplet localization to prospore membrane leading edge [GO:0140043], lipopolysaccharide localization to cell outer membrane [GO:0140334]